{
  "term_id": "GO:0005525",
  "gene_name": "Ras-related protein Rab-37",
  "gene": "UniProtKB:Q96AX2",
  "term_label": "GTP binding",
  "gene_symbol": "RAB37"
}